long-chain fatty acid [acyl-carrier-protein] ligase activity [GO:0008922] (molecular function) Relationships: is a type of fatty acid ligase activity [GO:0015645] Definition: Catalysis of the reaction: a long-chain fatty acid + ATP + holo-[ACP] = a long-chain fatty acyl-[ACP] + AMP + diphosphate. A long-chain fatty acid has an aliphatic tail containing 13 to 22 carbons. Also known as: acyl-acyl carrier protein synthetase, acyl-ACP synthetase activity, long-chain fatty acid-[acyl-carrier-protein] ligase activity, long-chain-fatty-acid-ACP ligase activity, long-chain-fatty-acid-[acyl-carrier protein] ligase activity, long-chain-fatty-acid-[acyl-carrier-protein] ligase activity, acyl-[acyl-carrier-protein] synthetase activity, acyl-acyl-carrier-protein synthetase activity, acyl-acyl-carrier-proteinsynthetase activity, long-chain-fatty-acid-acyl-carrier-protein ligase activity, long-chain-fatty-acid:acyl-carrier-protein ligase (AMP-forming) activity, stearoyl-ACP synthetase activity Note: While there is not universal consensus on the lengths of short-, medium-, long- and very-long-chain fatty acids, the GO uses the definitions in ChEBI (see CHEBI:26666, CHEBI:59554, CHEBI:15904 and CHEBI:27283). Sources: EC:6.2.1.20